oocyte localization involved in germarium-derived egg chamber formation [GO:0030720] (biological process) Also known as: establishment and maintenance of oocyte localization in egg chamber, establishment and maintenance of oocyte position during oogenesis, oocyte localisation involved in germarium-derived egg chamber formation, oogenesis, establishment and maintenance of oocyte localization, oogenesis, oocyte localization, oocyte positioning during oogenesis, oocyte localization during germarium-derived egg chamber formation, oocyte localization during oogenesis Definition: Directed movement of the oocyte, following its specification, from its original central position in the cyst to a posterior position relative to the nurse cells of the egg chamber, and its maintenance in this posterior location. This is the first sign of anterior-posterior asymmetry in the developing egg chamber. References: PMID:10449356 Sources: GOC:mtg_sensu Relationships: is a type of GO:0051674; is part of germarium-derived egg chamber formation [GO:0007293]